{
  "term_label": "mitochondrion",
  "gene": "UniProtKB:Q9NVA1",
  "term_id": "GO:0005739",
  "gene_symbol": "UQCC1",
  "gene_name": "Ubiquinol-cytochrome-c reductase complex assembly factor 1"
}